{
  "gene_symbol": "THNSL1",
  "term_label": "cytoplasm",
  "gene": "UniProtKB:Q8IYQ7",
  "term_id": "GO:0005737",
  "gene_name": "Threonine synthase-like 1"
}